{
  "term_id": "GO:0071914",
  "gene_symbol": "PROM2",
  "gene": "UniProtKB:Q8N271",
  "gene_name": "Prominin-2",
  "term_label": "prominosome"
}